{
  "gene_symbol": "CSRP2",
  "term_label": "sarcomere organization",
  "term_id": "GO:0045214",
  "gene": "UniProtKB:Q16527",
  "gene_name": "Cysteine and glycine-rich protein 2"
}